{
  "gene_name": "UDP-N-acetylglucosamine_UDP-glucose_GDP-mannose transporter",
  "term_id": "GO:0005462",
  "gene_symbol": "SLC35D2",
  "gene": "UniProtKB:Q76EJ3",
  "term_label": "UDP-N-acetylglucosamine transmembrane transporter activity"
}